{
  "term_label": "transcription coactivator activity",
  "gene_symbol": "CCDC124",
  "term_id": "GO:0003713",
  "gene_name": "Coiled-coil domain-containing protein 124",
  "gene": "UniProtKB:Q96CT7"
}